mesonephric proximal tubule development [GO:0061275] (biological process) Sources: GOC:mtg_kidney_jan10 Definition: The progression of the mesonephric proximal tubule over time, from its formation to the mature structure. The mesonephric proximal tubule extends from the capsule to the distal tubule. Relationships: is a type of mesonephric nephron tubule development [GO:0061242]; is a type of proximal tubule development [GO:0072014]